trophoblast cell migration [GO:0061450] (biological process) Sources: GOC:dph Definition: Trophoblast cell migration that is accomplished by extension and retraction of a pseudopodium. Trophoblast cells line the outside of the blastocyst. Regulation: regulated by regulation of trophoblast cell migration [GO:1901163]; negatively regulated by GO:1901164; positively regulated by positive regulation of trophoblast cell migration [GO:1901165] Relationships: is_a ameboidal-type cell migration [GO:0001667]; is part of embryo implantation [GO:0007566]